{
  "gene": "UniProtKB:Q8IVS2",
  "term_id": "GO:0006633",
  "gene_name": "Malonyl-CoA-acyl carrier protein transacylase, mitochondrial",
  "gene_symbol": "MCAT",
  "term_label": "fatty acid biosynthetic process"
}